{
  "gene": "UniProtKB:P54851",
  "gene_symbol": "EMP2",
  "gene_name": "Epithelial membrane protein 2",
  "term_id": "GO:0007155",
  "term_label": "cell adhesion"
}